plastid organization [GO:0009657] (BP) Relationships: is a type of organelle organization [GO:0006996] Also known as: plastid organisation, plastid organization and biogenesis Sources: GOC:mah Subtypes: GO:0009658, leucoplast organization [GO:0009659], amyloplast organization [GO:0009660], chromoplast organization [GO:0009661], etioplast organization [GO:0009662], plastid inheritance [GO:0009665], GO:0010111, plastid translation [GO:0032544] Definition: A process that is carried out at the cellular level which results in the assembly, arrangement of constituent parts, or disassembly of a plastid.